{
  "term_id": "UNKNOWN:0003",
  "gene_symbol": "TRAJ11",
  "gene_name": "T cell receptor alpha joining 11 (Fragment)",
  "term_label": "Unknown cellular component",
  "gene": "UniProtKB:A0A075B6Y8"
}